{
  "gene_symbol": "ST14",
  "gene": "UniProtKB:Q9Y5Y6",
  "term_id": "GO:0030216",
  "term_label": "keratinocyte differentiation",
  "gene_name": "Suppressor of tumorigenicity 14 protein"
}